{
  "gene": "UniProtKB:O95393",
  "term_label": "cytokine activity",
  "term_id": "GO:0005125",
  "gene_name": "Bone morphogenetic protein 10",
  "gene_symbol": "BMP10"
}